{
  "gene_name": "Protein ECT2",
  "gene": "UniProtKB:Q9H8V3",
  "term_id": "GO:0005634",
  "gene_symbol": "ECT2",
  "term_label": "nucleus"
}